{
  "gene_name": "Putative POM121-like protein 1-like",
  "term_label": "Unknown biological process",
  "term_id": "UNKNOWN:0002",
  "gene": "UniProtKB:A6NNC1",
  "gene_symbol": "A6NNC1"
}